{
  "gene_name": "C-C chemokine receptor-like 2",
  "gene_symbol": "CCRL2",
  "term_id": "GO:0006954",
  "gene": "UniProtKB:O00421",
  "term_label": "inflammatory response"
}